symbiont entry into host cell via permeabilization of endosomal membrane [GO:0099006] (biological process) Definition: The entry of a symbiont into a host cell, following endocytosis, via permeabilization of the endosomal membrane by membrane penetration protein(s) of the symbiont. This process mediates the entry of some non-enveloped virus into eukaryotic cells. In some cases, viral membrane-penetration protein requires to be activated to display its membrane penetrating activity. Activation can be due to receptor binding or the acidic pH of the endosomal lumen. Also known as: viral entry via permeabilization of endosomal membrane Relationships: is a type of GO:0140267 References: PMID:15329727, PMID:25055856